{
  "gene": "UniProtKB:Q13536",
  "term_label": "Unknown cellular component",
  "gene_symbol": "MIR9-1HG",
  "gene_name": "Protein CROC-4",
  "term_id": "UNKNOWN:0003"
}